{
  "gene_name": "E3 SUMO-protein ligase ZBED1",
  "term_label": "nucleus",
  "gene_symbol": "ZBED1",
  "term_id": "GO:0005634",
  "gene": "UniProtKB:O96006"
}